{
  "gene_symbol": "DPY19L2P1",
  "term_id": "UNKNOWN:0001",
  "gene_name": "Putative C-mannosyltransferase DPY19L2P1",
  "term_label": "Unknown molecular function",
  "gene": "UniProtKB:Q6NXN4"
}